{
  "gene_symbol": "RICTOR",
  "term_label": "TORC2 complex",
  "gene_name": "Rapamycin-insensitive companion of mTOR",
  "gene": "UniProtKB:Q6R327",
  "term_id": "GO:0031932"
}